{
  "gene_symbol": "CAP2",
  "gene_name": "Adenylyl cyclase-associated protein 2",
  "gene": "UniProtKB:P40123",
  "term_label": "adenylate cyclase binding",
  "term_id": "GO:0008179"
}